{
  "term_id": "GO:1990246",
  "gene": "UniProtKB:Q9H4I9",
  "gene_symbol": "SMDT1",
  "term_label": "uniplex complex",
  "gene_name": "Essential MCU regulator, mitochondrial"
}